{
  "term_label": "Unknown molecular function",
  "gene_name": "Protein jagunal homolog 1",
  "gene_symbol": "JAGN1",
  "gene": "UniProtKB:Q8N5M9",
  "term_id": "UNKNOWN:0001"
}